plant organ development [GO:0099402] (biological process) Definition: Development of a plant organ, a multi-tissue plant structure that forms a functional unit. Relationships: is a type of GO:0048856; is part of system development [GO:0048731] Also known as: development of a plant organ Subtypes: leaf formation [GO:0010338], root development [GO:0048364], GO:0048437, plant ovule development [GO:0048481], phyllome development [GO:0048827], post-embryonic plant organ development [GO:0090696] Sources: GOC:dos